response to statin [GO:0036273] (biological process) Also known as: response to HMG-CoA reductase inhibitor, response to hydroxymethylglutaryl-CoA reductase inhibitor Subtypes: GO:1903491 Definition: Any process that results in a change in state or activity of a cell or an organism (in terms of movement, secretion, enzyme production, gene expression, etc.) as a result of a statin stimulus. Statins are organooxygen compounds whose structure is related to compactin (mevastatin) and which may be used as an anticholesteremic drug due its EC:1.1.1.34/EC:1.1.1.88 (hydroxymethylglutaryl-CoA reductase) inhibitory properties. Note: Note that this term is in the subset of terms that should not be used for direct manual annotation of gene products. It was created to be used for cross-referencing by other ontologies. Direct annotations to this term may be amended during annotation QC. Sources: GOC:hp Relationships: is a type of response to oxygen-containing compound [GO:1901700]